{
  "gene": "UniProtKB:Q9GZW5",
  "gene_symbol": "SCAND2P",
  "term_label": "Unknown molecular function",
  "gene_name": "Putative SCAN domain-containing protein SCAND2P",
  "term_id": "UNKNOWN:0001"
}